positive regulation of somatostatin secretion [GO:0090274] (BP) Sources: GOC:BHF Definition: Any process that increases the rate, frequency, extent of the regulated release of somatostatin from secretory granules in the D cells of the pancreas. Relationships: is_a GO:0090273; is a type of GO:0090277; positively regulates GO:0070253